{
  "term_id": "UNKNOWN:0001",
  "gene_name": "Endoplasmic reticulum metallopeptidase 1",
  "term_label": "Unknown molecular function",
  "gene": "UniProtKB:Q7Z2K6",
  "gene_symbol": "ERMP1"
}